{
  "gene_name": "WASH complex subunit 5",
  "term_id": "UNKNOWN:0001",
  "gene": "UniProtKB:Q12768",
  "term_label": "Unknown molecular function",
  "gene_symbol": "WASHC5"
}